{
  "term_id": "GO:0003823",
  "gene_symbol": "IGHV1-38-4",
  "gene": "UniProtKB:P0DTW3",
  "gene_name": "Probable non-functional immunoglobulin heavy variable 1-38-4",
  "term_label": "antigen binding"
}